{
  "gene_name": "Neurabin-1",
  "gene": "UniProtKB:Q9ULJ8",
  "gene_symbol": "PPP1R9A",
  "term_label": "dendrite",
  "term_id": "GO:0030425"
}